protein farnesylation [GO:0018343] (biological process) Also known as: protein amino acid farnesylation, C-terminal protein farnesylation Sources: GOC:jl Relationships: is a type of protein prenylation [GO:0018342] Definition: The covalent attachment of a farnesyl group to a protein.